type II interferon production [GO:0032609] (biological process) Relationships: is a type of GO:0001816 References: PMID:15546383 Sources: GOC:add, GOC:mah Regulation: regulated by regulation of type II interferon production [GO:0032649]; negatively regulated by negative regulation of type II interferon production [GO:0032689]; positively regulated by positive regulation of type II interferon production [GO:0032729] Definition: The appearance of interferon-gamma due to biosynthesis or secretion following a cellular stimulus, resulting in an increase in its intracellular or extracellular levels. Interferon-gamma is also known as type II interferon. Also known as: IFNG production, interferon-gamma production, type II IFN production, interferon-gamma biosynthetic process, interferon-gamma secretion